{
  "term_label": "Unknown biological process",
  "gene_symbol": "LINC00311",
  "term_id": "UNKNOWN:0002",
  "gene_name": "Putative uncharacterized protein encoded by LINC00311",
  "gene": "UniProtKB:Q8N616"
}